{
  "term_id": "GO:0042147",
  "term_label": "retrograde transport, endosome to Golgi",
  "gene_symbol": "TMEM87A",
  "gene_name": "Transmembrane protein 87A",
  "gene": "UniProtKB:Q8NBN3"
}